{
  "term_id": "GO:0006355",
  "term_label": "regulation of DNA-templated transcription",
  "gene": "UniProtKB:Q92785",
  "gene_name": "Zinc finger protein ubi-d4",
  "gene_symbol": "DPF2"
}